RNA folding [GO:0034337] (biological process) Subtypes: tRNA folding [GO:0061818] Definition: The process of assisting in the covalent and noncovalent assembly of single or multimeric RNAs into the correct tertiary structure. Relationships: is a type of GO:0009987 References: PMID:10393192 Sources: GOC:mah Also known as: RNA chaperone